regulation of receptor recycling [GO:0001919] (biological process) Subtypes: GO:0001920, positive regulation of receptor recycling [GO:0001921] Definition: Any process that modulates the frequency, rate, or extent of receptor recycling. Sources: GOC:add Relationships: is a type of regulation of signaling [GO:0023051]; is a type of GO:0060255; regulates receptor recycling [GO:0001881]